{
  "gene_symbol": "GUCA1B",
  "gene": "UniProtKB:Q9UMX6",
  "term_id": "GO:0001917",
  "term_label": "photoreceptor inner segment",
  "gene_name": "Guanylyl cyclase-activating protein 2"
}